{
  "gene_name": "Hypoxia up-regulated protein 1",
  "gene": "UniProtKB:Q9Y4L1",
  "term_label": "negative regulation of hypoxia-induced intrinsic apoptotic signaling pathway",
  "term_id": "GO:1903298",
  "gene_symbol": "HYOU1"
}